negative regulation of synaptic vesicle recycling [GO:1903422] (biological process) Also known as: down regulation of synaptic vesicle recycling, down-regulation of synaptic vesicle recycling, downregulation of synaptic vesicle recycling, down regulation of kiss-and-run synaptic vesicle recycling, down regulation of kiss-and-stay synaptic vesicle recycling, down-regulation of kiss-and-run synaptic vesicle recycling, down-regulation of kiss-and-stay synaptic vesicle recycling, downregulation of kiss-and-run synaptic vesicle recycling, downregulation of kiss-and-stay synaptic vesicle recycling, inhibition of kiss-and-run synaptic vesicle recycling, inhibition of kiss-and-stay synaptic vesicle recycling, inhibition of synaptic vesicle recycling, negative regulation of kiss-and-run synaptic vesicle recycling, negative regulation of kiss-and-stay synaptic vesicle recycling Relationships: is a type of negative regulation of transport [GO:0051051]; is a type of regulation of synaptic vesicle recycling [GO:1903421]; RO_0002212 synaptic vesicle recycling [GO:0036465] References: PMID:22745285 Sources: GOC:PARL, GOC:TermGenie, GOC:pad, GO_REF:0000058 Note: An example of this is mouse LRRK2 (Q5S006) in PMID:21307259 inferred from mutant phenotype Definition: Any process that stops, prevents or reduces the frequency, rate or extent of synaptic vesicle recycling. Subtypes: negative regulation of synaptic vesicle endocytosis [GO:1900243]